positive regulation of translation, ncRNA-mediated [GO:0045975] (biological process) Definition: Any process, mediated by small non-coding RNAs, that activates or increases the rate that mRNAs are effectively translated into protein. Sources: GOC:dph, GOC:go_curators, GOC:tb Also known as: up regulation of mRNA translation, ncRNA-mediated, up-regulation of mRNA translation, ncRNA-mediated, upregulation of mRNA translation, ncRNA-mediated, activation of mRNA translation, ncRNA-mediated, stimulation of mRNA translation, ncRNA-mediated Relationships: is_a positive regulation of translation [GO:0045727]; is a type of regulation of translation, ncRNA-mediated [GO:0045974]